mesodermal cell fate commitment [GO:0001710] (biological process) Definition: The cell differentiation process that results in commitment of a cell to become part of the mesoderm. Sources: GOC:go_curators, ISBN:0878932437 Also known as: mesoderm cell fate commitment Relationships: is a type of cell fate commitment involved in formation of primary germ layer [GO:0060795]; is part of mesodermal cell differentiation [GO:0048333] Subtypes: GO:0048322, paraxial mesodermal cell fate commitment [GO:0048343], GO:0048372, intermediate mesodermal cell fate commitment [GO:0048393]